{
  "gene_name": "Inositol 1,4,5-trisphosphate receptor type 3",
  "gene_symbol": "ITPR3",
  "term_label": "phosphatidylinositol binding",
  "term_id": "GO:0035091",
  "gene": "UniProtKB:Q14573"
}